{
  "gene_symbol": "SNX12",
  "gene": "UniProtKB:Q9UMY4",
  "term_label": "phosphatidylinositol-3-phosphate binding",
  "term_id": "GO:0032266",
  "gene_name": "Sorting nexin-12"
}